{
  "gene_name": "Dolichol-phosphate mannosyltransferase subunit 3",
  "term_id": "GO:0033185",
  "term_label": "dolichol-phosphate-mannose synthase complex",
  "gene": "UniProtKB:Q9P2X0",
  "gene_symbol": "DPM3"
}